{
  "gene_symbol": "RRAGB",
  "term_label": "GTP binding",
  "gene": "UniProtKB:Q5VZM2",
  "term_id": "GO:0005525",
  "gene_name": "Ras-related GTP-binding protein B"
}